tRNA dihydrouridine synthesis [GO:0002943] (biological process) Definition: The process whereby a uridine in a transfer RNA is converted to dihydrouridine. Sources: GOC:hjd, ISBN:155581073X Note: Dihydrouridine is found in numerous positions within loop I, the so-called dihydrouridine loop, of many transfer RNAs. Most often found at positions 16 and 17, but also sometimes at positions 20, 20a, and 20b. Relationships: is_a tRNA modification [GO:0006400]